{
  "term_label": "regulation of transcription by RNA polymerase II",
  "gene": "UniProtKB:Q8N0Y2",
  "gene_name": "Zinc finger protein 444",
  "term_id": "GO:0006357",
  "gene_symbol": "ZNF444"
}